{
  "gene_symbol": "MT-ND1",
  "gene_name": "NADH-ubiquinone oxidoreductase chain 1",
  "gene": "UniProtKB:P03886",
  "term_label": "NADH dehydrogenase activity",
  "term_id": "GO:0003954"
}